{
  "gene": "UniProtKB:P25800",
  "term_label": "positive regulation of transcription by RNA polymerase II",
  "gene_symbol": "LMO1",
  "gene_name": "Rhombotin-1",
  "term_id": "GO:0045944"
}